{
  "gene_name": "UV excision repair protein RAD23 homolog B",
  "gene": "UniProtKB:P54727",
  "gene_symbol": "RAD23B",
  "term_label": "cytosol",
  "term_id": "GO:0005829"
}